retinoic acid receptor signaling pathway [GO:0048384] (biological process) Also known as: RAR signaling pathway, nuclear receptor-mediated retinoic acid signaling pathway, retinoic acid receptor signalling pathway Relationships: is_a GO:0009755; is_a nuclear receptor-mediated signaling pathway [GO:0141193] Regulation: regulated by regulation of retinoic acid receptor signaling pathway [GO:0048385]; positively regulated by positive regulation of retinoic acid receptor signaling pathway [GO:0048386]; negatively regulated by GO:0048387 Sources: GOC:dgh Definition: A nuclear receptor-mediated signaling pathway initiated by a retinoic acid binding to an intracellular receptor of the nuclear receptor protein family, and ending with regulation of a downstream cellular process, e.g. transcription.